{
  "term_label": "calcium ion transport",
  "gene_symbol": "CACNB2",
  "term_id": "GO:0006816",
  "gene_name": "Voltage-dependent L-type calcium channel subunit beta-2",
  "gene": "UniProtKB:Q08289"
}